{
  "gene": "UniProtKB:Q96IT1",
  "term_id": "GO:0000978",
  "gene_name": "Zinc finger protein 496",
  "term_label": "RNA polymerase II cis-regulatory region sequence-specific DNA binding",
  "gene_symbol": "ZNF496"
}